{
  "term_id": "GO:0005544",
  "term_label": "calcium-dependent phospholipid binding",
  "gene_symbol": "ESYT3",
  "gene": "UniProtKB:A0FGR9",
  "gene_name": "Extended synaptotagmin-3"
}